regulation of sclerotium development [GO:1901922] (biological process) Definition: Any process that modulates the frequency, rate or extent of sclerotium development. References: PMID:21148914 Sources: GOC:TermGenie, GOC:di Subtypes: negative regulation of sclerotium development [GO:1901923], positive regulation of sclerotium development [GO:1901924] Relationships: is a type of regulation of developmental process [GO:0050793]; regulates GO:1990045